{
  "gene": "UniProtKB:Q9H944",
  "gene_name": "Mediator of RNA polymerase II transcription subunit 20",
  "term_id": "GO:0006357",
  "gene_symbol": "MED20",
  "term_label": "regulation of transcription by RNA polymerase II"
}